{
  "term_label": "apical plasma membrane",
  "gene_name": "Sodium-dependent phosphate transport protein 3",
  "term_id": "GO:0016324",
  "gene": "UniProtKB:O00624",
  "gene_symbol": "SLC17A2"
}